{
  "gene_name": "Laminin subunit alpha-1",
  "term_id": "GO:0007399",
  "term_label": "nervous system development",
  "gene": "UniProtKB:P25391",
  "gene_symbol": "LAMA1"
}